{
  "gene_symbol": "GPD1L",
  "term_id": "UNKNOWN:0002",
  "gene_name": "Glycerol-3-phosphate dehydrogenase 1-like protein",
  "term_label": "Unknown biological process",
  "gene": "UniProtKB:Q8N335"
}